{
  "gene": "UniProtKB:O95299",
  "gene_symbol": "NDUFA10",
  "term_id": "GO:0045271",
  "gene_name": "NADH dehydrogenase [ubiquinone] 1 alpha subcomplex subunit 10, mitochondrial",
  "term_label": "respiratory chain complex I"
}